{
  "term_label": "endosome organization",
  "gene_symbol": "USP50",
  "gene": "UniProtKB:Q70EL3",
  "gene_name": "Inactive ubiquitin carboxyl-terminal hydrolase 50",
  "term_id": "GO:0007032"
}